death receptor activity [GO:0005035] (molecular function) Definition: Combining with an extracellular messenger (called a death ligand), and transmitting the signal from one side of the plasma membrane to the other to initiate apoptotic or necrotic cell death. Subtypes: tumor necrosis factor receptor activity [GO:0005031], TRAIL receptor activity [GO:0036463] Also known as: apoptosis-activating receptor activity Relationships: is a type of transmembrane signaling receptor activity [GO:0004888]; BFO_0000050 GO:0012501 Regulation: positively regulated by death receptor agonist activity [GO:0038177] References: PMID:10209153 Sources: GOC:BHF, GOC:bf, GOC:ecd, GOC:mtg_apoptosis, GOC:rl